{
  "term_id": "GO:0000981",
  "gene_symbol": "SP7",
  "gene_name": "Transcription factor Sp7",
  "term_label": "DNA-binding transcription factor activity, RNA polymerase II-specific",
  "gene": "UniProtKB:Q8TDD2"
}